{
  "gene_symbol": "MMACHC",
  "term_id": "GO:0032451",
  "term_label": "demethylase activity",
  "gene_name": "Cyanocobalamin reductase _ alkylcobalamin dealkylase",
  "gene": "UniProtKB:Q9Y4U1"
}